{
  "gene_name": "Pregnancy-specific beta-1-glycoprotein 6",
  "gene_symbol": "PSG6",
  "gene": "UniProtKB:Q00889",
  "term_id": "UNKNOWN:0002",
  "term_label": "Unknown biological process"
}